{
  "gene": "UniProtKB:Q8NFJ6",
  "gene_name": "Prokineticin receptor 2",
  "term_id": "GO:0007623",
  "gene_symbol": "PROKR2",
  "term_label": "circadian rhythm"
}